hormonal regulation of the force of heart contraction [GO:0003058] (biological process) Relationships: is a type of regulation of the force of heart contraction by chemical signal [GO:0003057] Definition: The process in which the hormones modulates the force of heart muscle contraction. A hormone is one of a group of substances formed in very small amounts in one specialized organ or group of cells and carried (sometimes in the bloodstream) to another organ or group of cells, in the same organism, upon which they have a specific regulatory action. Also known as: hormonal cardiac inotropy, hormonal regulation of the force of heart muscle contraction Sources: GOC:mtg_cardio, GOC:rl